{
  "term_id": "GO:0005337",
  "gene_name": "Equilibrative nucleoside transporter 2",
  "gene_symbol": "SLC29A2",
  "gene": "UniProtKB:Q14542",
  "term_label": "nucleoside transmembrane transporter activity"
}